{
  "gene_symbol": "KCNJ10",
  "term_label": "Unknown molecular function",
  "term_id": "UNKNOWN:0001",
  "gene_name": "ATP-sensitive inward rectifier potassium channel 10",
  "gene": "UniProtKB:P78508"
}